{
  "gene": "UniProtKB:Q8N8E2",
  "gene_name": "Zinc finger protein 513",
  "term_label": "DNA-binding transcription factor activity",
  "gene_symbol": "ZNF513",
  "term_id": "GO:0003700"
}